rescue of stalled ribosome [GO:0072344] (biological process) Relationships: is a type of translational elongation [GO:0006414]; is a type of ribosome disassembly [GO:0032790] References: PMID:18557701, PMID:19170872, PMID:20117091, PMID:20185543 Sources: GOC:jh2, GOC:mah Definition: A process of translational elongation that takes place when a ribosome has stalled during translation, and results in freeing the ribosome from the stalled translation complex. Subtypes: trans-translation-dependent protein tagging [GO:0070930], protein-RNA covalent cross-linking repair [GO:0160127]